{
  "term_label": "RNA polymerase II cis-regulatory region sequence-specific DNA binding",
  "term_id": "GO:0000978",
  "gene": "UniProtKB:Q96T92",
  "gene_name": "Insulinoma-associated protein 2",
  "gene_symbol": "INSM2"
}